{
  "term_label": "calcium-dependent protein binding",
  "term_id": "GO:0048306",
  "gene_symbol": "S100A4",
  "gene_name": "Protein S100-A4",
  "gene": "UniProtKB:P26447"
}